{
  "term_id": "GO:0006896",
  "gene": "UniProtKB:O43747",
  "gene_name": "AP-1 complex subunit gamma-1",
  "term_label": "Golgi to vacuole transport",
  "gene_symbol": "AP1G1"
}